{
  "term_label": "positive regulation of T cell activation",
  "gene": "UniProtKB:P05538",
  "gene_symbol": "HLA-DQB2",
  "term_id": "GO:0050870",
  "gene_name": "HLA class II histocompatibility antigen, DQ beta 2 chain"
}